{
  "term_label": "nucleus",
  "gene": "UniProtKB:P43364",
  "gene_symbol": "MAGEA11",
  "gene_name": "Melanoma-associated antigen 11",
  "term_id": "GO:0005634"
}